{
  "gene_symbol": "NR1D2",
  "gene": "UniProtKB:Q14995",
  "term_label": "cell differentiation",
  "gene_name": "Nuclear receptor subfamily 1 group D member 2",
  "term_id": "GO:0030154"
}